acquisition of nutrients from symbiont [GO:0051850] (biological process) Definition: The production of structures and/or molecules in an organism that are required for the acquisition and/or utilization of nutrients obtained from its symbiont organism. The symbiont is defined as the smaller of the organisms involved in a symbiotic interaction. Sources: GOC:cc Relationships: is a type of GO:0051702